laminin-15 complex [GO:1990340] (cellular component) References: PMID:17453709 Sources: GOC:bhm Relationships: is a type of laminin complex [GO:0043256] Also known as: laminin-523 Definition: A laminin complex composed of alpha5, beta2 and gamma3 polypeptide chains.